{
  "gene_name": "Actin, cytoplasmic 2",
  "gene": "UniProtKB:P63261",
  "gene_symbol": "ACTG1",
  "term_id": "GO:0015629",
  "term_label": "actin cytoskeleton"
}